{
  "gene_symbol": "TEKT1",
  "term_label": "microtubule cytoskeleton",
  "term_id": "GO:0015630",
  "gene_name": "Tektin-1",
  "gene": "UniProtKB:Q969V4"
}